{
  "term_label": "Unknown molecular function",
  "gene_name": "Zinc finger and BTB domain-containing protein 44",
  "gene": "UniProtKB:Q8NCP5",
  "gene_symbol": "ZBTB44",
  "term_id": "UNKNOWN:0001"
}